{
  "gene_symbol": "OPN1MW3",
  "gene_name": "Medium-wave-sensitive opsin 3",
  "gene": "UniProtKB:P0DN78",
  "term_label": "plasma membrane",
  "term_id": "GO:0005886"
}